{
  "gene": "UniProtKB:Q5JWF8",
  "term_id": "GO:0005200",
  "gene_name": "Actin-like protein 10",
  "term_label": "structural constituent of cytoskeleton",
  "gene_symbol": "ACTL10"
}